{
  "term_id": "GO:0030198",
  "gene_name": "SPARC-related modular calcium-binding protein 2",
  "gene": "UniProtKB:Q9H3U7",
  "term_label": "extracellular matrix organization",
  "gene_symbol": "SMOC2"
}